{
  "gene_name": "Sodium_hydrogen exchanger 8",
  "gene": "UniProtKB:Q9Y2E8",
  "gene_symbol": "SLC9A8",
  "term_label": "regulation of intracellular pH",
  "term_id": "GO:0051453"
}